{
  "term_id": "GO:0005886",
  "gene_name": "Olfactory receptor 52N4",
  "term_label": "plasma membrane",
  "gene_symbol": "OR52N4",
  "gene": "UniProtKB:Q8NGI2"
}